{
  "term_label": "microtubule binding",
  "gene_symbol": "MAPT",
  "term_id": "GO:0008017",
  "gene": "UniProtKB:P10636",
  "gene_name": "Microtubule-associated protein tau"
}